{
  "term_id": "GO:0014069",
  "term_label": "postsynaptic density",
  "gene_symbol": "SHISA6",
  "gene": "UniProtKB:Q6ZSJ9",
  "gene_name": "Protein shisa-6"
}